{
  "gene_symbol": "C1QTNF3",
  "term_label": "synaptic cleft",
  "term_id": "GO:0043083",
  "gene": "UniProtKB:Q9BXJ4",
  "gene_name": "Complement C1q tumor necrosis factor-related protein 3"
}